proteasome storage granule assembly [GO:1902906] (biological process) Relationships: is_a membraneless organelle assembly [GO:0140694] References: PMID:23690178 Sources: GOC:TermGenie, GOC:di, GO_REF:0000079 Definition: The aggregation, arrangement and bonding together of a set of components to form a proteasome storage granule. Also known as: proteasome storage granule formation, sequestration of proteasome core complex in proteasome storage granule, PSG assembly, PSG formation